{
  "term_label": "Unknown cellular component",
  "term_id": "UNKNOWN:0003",
  "gene_name": "Dolichyl-diphosphooligosaccharide--protein glycosyltransferase subunit STT3A",
  "gene": "UniProtKB:P46977",
  "gene_symbol": "STT3A"
}